{
  "gene_symbol": "RASGRF1",
  "gene": "UniProtKB:Q13972",
  "gene_name": "Ras-specific guanine nucleotide-releasing factor 1",
  "term_id": "GO:0005886",
  "term_label": "plasma membrane"
}